{
  "gene_name": "Cancer_testis antigen family 45 member A8",
  "gene": "UniProtKB:P0DMV1",
  "term_id": "UNKNOWN:0001",
  "gene_symbol": "CT45A8",
  "term_label": "Unknown molecular function"
}